regulation of ergosterol biosynthetic process [GO:0032443] (biological process) Subtypes: GO:0010895, positive regulation of ergosterol biosynthetic process [GO:0070452] Relationships: is a type of regulation of sterol biosynthetic process [GO:0106118]; is a type of regulation of alcohol biosynthetic process [GO:1902930]; regulates ergosterol biosynthetic process [GO:0006696] Sources: GOC:mah Definition: Any process that modulates the frequency, rate or extent of the chemical reactions and pathways resulting in the formation of ergosterol.